lymphocyte chemotaxis across high endothelial venule [GO:0002518] (BP) Definition: The movement of a lymphocyte to cross a high endothelial venule in response to an external stimulus. References: PMID:15122201 Sources: GOC:add, ISBN:0781735149 Relationships: is a type of lymphocyte chemotaxis [GO:0048247] Subtypes: B cell chemotaxis across high endothelial venule [GO:0035769]